{
  "gene": "UniProtKB:Q9Y2L8",
  "term_id": "GO:0000981",
  "term_label": "DNA-binding transcription factor activity, RNA polymerase II-specific",
  "gene_name": "Zinc finger protein with KRAB and SCAN domains 5",
  "gene_symbol": "ZKSCAN5"
}